{
  "gene_name": "Cell division cycle protein 27 homolog",
  "gene_symbol": "CDC27",
  "term_label": "anaphase-promoting complex-dependent catabolic process",
  "term_id": "GO:0031145",
  "gene": "UniProtKB:P30260"
}